precorrin-8X methylmutase activity [GO:0016993] (MF) Also known as: precorrin-8X 11,12-methylmutase activity, hydrogenobyrinic acid-binding protein activity, HBA synthase activity, precorrin isomerase activity Definition: Catalysis of the reaction: precorrin-8X = hydrogenobyrinate. Relationships: is a type of intramolecular acyltransferase activity [GO:0016867] Sources: EC:5.4.99.61